beta-galactofuranosidase activity [GO:0033944] (molecular function) Also known as: beta-D-galactofuranosidase activity, beta-D-galactofuranoside hydrolase activity, exo-beta-D-galactofuranosidase activity, exo-beta-galactofuranosidase activity Sources: EC:3.2.1.146 Definition: Catalysis of the hydrolysis of terminal non-reducing beta-D-galactofuranosides, releasing galactose. Relationships: is a type of GO:0004553